{
  "term_id": "GO:0098803",
  "gene_symbol": "COX7A2",
  "gene": "UniProtKB:P14406",
  "term_label": "respiratory chain complex",
  "gene_name": "Cytochrome c oxidase subunit 7A2, mitochondrial"
}